U1 snRNP [GO:0005685] (cellular component) Sources: GOC:krc, GOC:mah, ISBN:0879695897 Definition: A ribonucleoprotein complex that contains small nuclear RNA U1, a heptameric ring of Sm proteins, as well as several proteins that are unique to the U1 snRNP, most of which remain associated with the U1 snRNA both while the U1 snRNP is free or assembled into a series of spliceosomal complexes. Also known as: snRNP U1 Relationships: is a type of spliceosomal snRNP complex [GO:0097525]